{
  "gene": "UniProtKB:P00488",
  "gene_symbol": "F13A1",
  "term_label": "protein-glutamine gamma-glutamyltransferase activity",
  "gene_name": "Coagulation factor XIII A chain",
  "term_id": "GO:0003810"
}